{
  "term_label": "Unknown cellular component",
  "gene": "UniProtKB:Q6UXT8",
  "gene_name": "ALK and LTK ligand 1",
  "gene_symbol": "ALKAL1",
  "term_id": "UNKNOWN:0003"
}